{
  "gene_symbol": "EP400",
  "term_label": "chromatin binding",
  "term_id": "GO:0003682",
  "gene": "UniProtKB:Q96L91",
  "gene_name": "E1A-binding protein p400"
}